response to sodium arsenite [GO:1903935] (biological process) Subtypes: GO:1903936 References: PMID:18674524 Sources: GOC:TermGenie, GO_REF:0000071 Relationships: is a type of GO:0046685; is_a response to salt [GO:1902074] Definition: Any process that results in a change in state or activity of a cell or an organism (in terms of movement, secretion, enzyme production, gene expression, etc.) as a result of a sodium arsenite stimulus.